{
  "term_id": "UNKNOWN:0002",
  "term_label": "Unknown biological process",
  "gene_symbol": "LOC122319696",
  "gene_name": "Uncharacterized protein",
  "gene": "UniProtKB:A0A590UK24"
}